{
  "gene_name": "ATP-dependent RNA helicase DHX30",
  "term_id": "GO:0003678",
  "gene": "UniProtKB:Q7L2E3",
  "gene_symbol": "DHX30",
  "term_label": "DNA helicase activity"
}